{
  "term_id": "UNKNOWN:0002",
  "term_label": "Unknown biological process",
  "gene_symbol": "ANKRD7",
  "gene": "UniProtKB:Q92527",
  "gene_name": "Ankyrin repeat domain-containing protein 7"
}